{
  "term_id": "UNKNOWN:0003",
  "gene": "UniProtKB:Q6ZT21",
  "gene_name": "Transmembrane protein with metallophosphoesterase domain",
  "gene_symbol": "TMPPE",
  "term_label": "Unknown cellular component"
}